{
  "gene_symbol": "TXNDC16",
  "gene_name": "Thioredoxin domain-containing protein 16",
  "term_label": "Unknown molecular function",
  "term_id": "UNKNOWN:0001",
  "gene": "UniProtKB:Q9P2K2"
}